regulation of plasmacytoid dendritic cell antigen processing and presentation [GO:0002610] (biological process) Definition: Any process that modulates the frequency, rate, or extent of plasmacytoid dendritic cell antigen processing and presentation. Sources: GOC:add Subtypes: negative regulation of plasmacytoid dendritic cell antigen processing and presentation [GO:0002611], positive regulation of plasmacytoid dendritic cell antigen processing and presentation [GO:0002612] Relationships: is_a GO:0002604; regulates GO:0002470